{
  "gene_symbol": "PIK3CG",
  "term_label": "plasma membrane",
  "term_id": "GO:0005886",
  "gene": "UniProtKB:P48736",
  "gene_name": "Phosphatidylinositol 4,5-bisphosphate 3-kinase catalytic subunit gamma isoform"
}